{
  "gene_symbol": "ZNRF2",
  "term_id": "GO:0016020",
  "gene": "UniProtKB:Q8NHG8",
  "term_label": "membrane",
  "gene_name": "E3 ubiquitin-protein ligase ZNRF2"
}